{
  "term_label": "negative regulation of execution phase of apoptosis",
  "gene_symbol": "MTRNR2L11",
  "gene_name": "Humanin-like 11",
  "term_id": "GO:1900118",
  "gene": "UniProtKB:S4R3Y5"
}